{
  "gene_name": "Pleckstrin homology domain-containing family A member 5",
  "gene": "UniProtKB:Q9HAU0",
  "term_id": "GO:0032266",
  "gene_symbol": "PLEKHA5",
  "term_label": "phosphatidylinositol-3-phosphate binding"
}